{
  "term_id": "GO:0042059",
  "gene_name": "E3 ubiquitin-protein ligase CBL-B",
  "term_label": "negative regulation of epidermal growth factor receptor signaling pathway",
  "gene": "UniProtKB:Q13191",
  "gene_symbol": "CBLB"
}